{
  "gene_symbol": "TRAV19",
  "term_id": "GO:0019814",
  "gene": "UniProtKB:A0A0A6YYK7",
  "gene_name": "T cell receptor alpha variable 19",
  "term_label": "immunoglobulin complex"
}